aryl-aldehyde dehydrogenase (NADP+) activity [GO:0047683] (molecular function) Sources: RHEA:19229 Relationships: is a type of aldehyde dehydrogenase (NADP+) activity [GO:0033721] Definition: Catalysis of the reaction: an aromatic aldehyde + NADP+ + AMP + diphosphate + H2O = an aromatic acid + NADPH + ATP. Also known as: aromatic acid reductase activity, aryl-aldehyde:NADP+ oxidoreductase (ATP-forming)